{
  "term_id": "UNKNOWN:0001",
  "gene": "UniProtKB:Q5T5Y3",
  "gene_name": "Calmodulin-regulated spectrin-associated protein 1",
  "term_label": "Unknown molecular function",
  "gene_symbol": "CAMSAP1"
}